{
  "gene_symbol": "DYNLT5",
  "term_id": "GO:0005868",
  "gene": "UniProtKB:Q8N7M0",
  "term_label": "cytoplasmic dynein complex",
  "gene_name": "Dynein light chain Tctex-type 5"
}